{
  "term_id": "GO:0003690",
  "term_label": "double-stranded DNA binding",
  "gene_name": "X-ray repair cross-complementing protein 5",
  "gene_symbol": "XRCC5",
  "gene": "UniProtKB:P13010"
}